anterior/posterior lineage restriction, imaginal disc [GO:0048099] (biological process) Definition: Formation and/or maintenance of a lineage boundary between anterior and posterior compartments that cells cannot cross, thus separating the populations of cells in each compartment. Subtypes: leg disc anterior/posterior lineage restriction [GO:0035201] Relationships: is a type of imaginal disc lineage restriction [GO:0035161]; is part of anterior/posterior pattern specification, imaginal disc [GO:0007448] References: PMID:10625531, PMID:9374402 Sources: GOC:jid